{
  "gene_symbol": "SMCR8",
  "gene_name": "Guanine nucleotide exchange protein SMCR8",
  "term_id": "UNKNOWN:0001",
  "gene": "UniProtKB:Q8TEV9",
  "term_label": "Unknown molecular function"
}